{
  "gene": "UniProtKB:Q96M94",
  "term_label": "nuclear protein quality control by the ubiquitin-proteasome system",
  "term_id": "GO:0071630",
  "gene_name": "Kelch-like protein 15",
  "gene_symbol": "KLHL15"
}